negative regulation of strand invasion [GO:0060543] (biological process) Relationships: is a type of negative regulation of DNA recombination [GO:0045910]; is a type of regulation of strand invasion [GO:0060542]; negatively regulates DNA strand invasion [GO:0042148] Sources: GOC:dph, GOC:elh, GOC:tb Definition: Any process that decreases the rate, frequency or extent of strand invasion. Strand invasion is the process in which the nucleoprotein complex (composed of the broken single-strand DNA and the recombinase) searches and identifies a region of homology in intact duplex DNA. The broken single-strand DNA displaces the like strand and forms Watson-Crick base pairs with its complement, forming a duplex in which each strand is from one of the two recombining DNA molecules. Also known as: negative regulation of Rad51-mediated strand invasion, negative regulation of D-loop biosynthesis, negative regulation of D-loop formation